{
  "gene_symbol": "KCNS3",
  "term_label": "voltage-gated potassium channel complex",
  "term_id": "GO:0008076",
  "gene_name": "Potassium voltage-gated channel subfamily S member 3",
  "gene": "UniProtKB:Q9BQ31"
}